lysophosphatidic acid acyltransferase activity [GO:0042171] (molecular function) References: PMID:16369050 Sources: GOC:ab Definition: Catalysis of the transfer of acyl groups from an acyl-CoA to lysophosphatidic acid to form phosphatidic acid. Subtypes: 1-acylglycerol-3-phosphate O-acyltransferase activity [GO:0003841], 2-acylglycerol-3-phosphate O-acyltransferase activity [GO:0047144] Relationships: is a type of GO:0071617 Also known as: LPAAT activity